positive regulation of hyphopodium formation [GO:0075189] (biological process) Relationships: is a type of positive regulation of developmental process [GO:0051094]; is a type of regulation of hyphopodium formation [GO:0075188]; RO_0002213 hyphopodium formation [GO:0075187] Sources: GOC:pamgo_curators Also known as: positive regulation of hyphopodium formation on or near host Definition: Any process that activates or increases the frequency, rate or extent of symbiont hyphopodium formation on or near its host organism. The host is defined as the larger of the organisms involved in a symbiotic interaction.